{
  "term_label": "Unknown molecular function",
  "gene": "UniProtKB:Q496H8",
  "term_id": "UNKNOWN:0001",
  "gene_symbol": "NRN1L",
  "gene_name": "Neuritin-like protein"
}